{
  "gene_symbol": "SPIRE1",
  "gene": "UniProtKB:Q08AE8",
  "term_label": "cytoplasmic vesicle membrane",
  "gene_name": "Protein spire homolog 1",
  "term_id": "GO:0030659"
}